{
  "term_id": "GO:0017080",
  "term_label": "sodium channel regulator activity",
  "gene_name": "Fibroblast growth factor 11",
  "gene_symbol": "FGF11",
  "gene": "UniProtKB:Q92914"
}